{
  "gene_name": "Alcohol dehydrogenase 1C",
  "gene_symbol": "ADH1C",
  "term_id": "GO:0042573",
  "term_label": "retinoic acid metabolic process",
  "gene": "UniProtKB:P00326"
}